2-alkyn-1-ol dehydrogenase activity [GO:0047535] (molecular function) Also known as: 2-butyne-1,4-diol:NAD+ 1-oxidoreductase activity Relationships: is a type of oxidoreductase activity, acting on the CH-OH group of donors, NAD or NADP as acceptor [GO:0016616] Sources: EC:1.1.1.165, RHEA:19101 Definition: Catalysis of the reaction: 2-butyne-1,4-diol + NAD+ = 4-hydroxy-2-butynal + H+ + NADH.